{
  "term_id": "GO:0080025",
  "gene": "UniProtKB:O75146",
  "gene_name": "Huntingtin-interacting protein 1-related protein",
  "gene_symbol": "HIP1R",
  "term_label": "phosphatidylinositol-3,5-bisphosphate binding"
}